{
  "gene_symbol": "ACOD1",
  "gene_name": "Cis-aconitate decarboxylase",
  "term_id": "GO:0006952",
  "gene": "UniProtKB:A6NK06",
  "term_label": "defense response"
}